{
  "gene": "UniProtKB:Q96JP2",
  "gene_symbol": "MYO15B",
  "gene_name": "Unconventional myosin-XVB",
  "term_id": "UNKNOWN:0002",
  "term_label": "Unknown biological process"
}